{
  "term_label": "cell differentiation",
  "term_id": "GO:0030154",
  "gene": "UniProtKB:Q14541",
  "gene_name": "Hepatocyte nuclear factor 4-gamma",
  "gene_symbol": "HNF4G"
}